{
  "term_label": "Unknown biological process",
  "gene": "UniProtKB:A6NKC0",
  "term_id": "UNKNOWN:0002",
  "gene_name": "Putative protein FAM90A7",
  "gene_symbol": "FAM90A7"
}